{
  "term_label": "Unknown biological process",
  "term_id": "UNKNOWN:0002",
  "gene": "UniProtKB:Q9UJT2",
  "gene_name": "Testis-specific serine kinase substrate",
  "gene_symbol": "TSKS"
}